{
  "gene_name": "Serglycin",
  "term_id": "GO:0030502",
  "gene_symbol": "SRGN",
  "term_label": "negative regulation of bone mineralization",
  "gene": "UniProtKB:P10124"
}